o-succinylbenzoate-CoA ligase activity [GO:0008756] (molecular function) Sources: EC:6.2.1.26 Definition: Catalysis of the reaction: 2-succinylbenzoate + ATP + CoA = 2-succinylbenzoyl-CoA + AMP + diphosphate. Relationships: is a type of CoA-ligase activity [GO:0016405]; is a type of GO:0016878 Also known as: 2-succinylbenzoate:CoA ligase (AMP-forming), OSB-CoA synthetase activity, o-succinylbenzoate:CoA ligase (AMP-forming), o-succinylbenzoyl-CoA synthetase activity, o-succinylbenzoyl-coenzyme A synthetase activity